{
  "term_label": "endosome",
  "term_id": "GO:0005768",
  "gene_name": "Target of Myb1 membrane trafficking protein",
  "gene_symbol": "TOM1",
  "gene": "UniProtKB:O60784"
}